{
  "gene": "UniProtKB:Q6ZU64",
  "gene_symbol": "CFAP65",
  "term_id": "GO:0036126",
  "term_label": "sperm flagellum",
  "gene_name": "Cilia- and flagella-associated protein 65"
}